{
  "term_label": "cholesterol biosynthetic process",
  "gene_name": "3-beta-hydroxysteroid-Delta(8),Delta(7)-isomerase",
  "term_id": "GO:0006695",
  "gene": "UniProtKB:Q15125",
  "gene_symbol": "EBP"
}